{
  "gene_symbol": "EIF3K",
  "gene": "UniProtKB:Q9UBQ5",
  "gene_name": "Eukaryotic translation initiation factor 3 subunit K",
  "term_label": "translation initiation factor activity",
  "term_id": "GO:0003743"
}